{
  "term_id": "UNKNOWN:0001",
  "gene": "UniProtKB:P11836",
  "term_label": "Unknown molecular function",
  "gene_symbol": "MS4A1",
  "gene_name": "B-lymphocyte antigen CD20"
}